{
  "gene": "UniProtKB:O15162",
  "term_id": "GO:0070782",
  "gene_symbol": "PLSCR1",
  "term_label": "phosphatidylserine exposure on apoptotic cell surface",
  "gene_name": "Phospholipid scramblase 1"
}